{
  "gene_name": "von Willebrand factor C domain-containing protein 2-like",
  "gene_symbol": "VWC2L",
  "term_label": "extracellular space",
  "term_id": "GO:0005615",
  "gene": "UniProtKB:B2RUY7"
}